triazole transport [GO:1901504] (biological process) Relationships: is a type of nitrogen compound transport [GO:0071705] Sources: GOC:TermGenie, GOC:pr Definition: The directed movement of a triazole into, out of or within a cell, or between cells, by means of some agent such as a transporter or pore.